{
  "term_id": "GO:0051123",
  "gene_name": "TATA-box binding protein associated factor 11 like protein 2",
  "gene": "UniProtKB:A6NLC8",
  "term_label": "RNA polymerase II preinitiation complex assembly",
  "gene_symbol": "TAF11L2"
}